positive regulation of myofibroblast differentiation [GO:1904762] (biological process) Also known as: positive regulation of myofibroblast cell differentiation, up regulation of myofibroblast cell differentiation, up regulation of myofibroblast differentiation, up-regulation of myofibroblast cell differentiation, up-regulation of myofibroblast differentiation, upregulation of myofibroblast cell differentiation, upregulation of myofibroblast differentiation, activation of myofibroblast cell differentiation, activation of myofibroblast differentiation Relationships: is a type of GO:0045597; is a type of regulation of myofibroblast differentiation [GO:1904760]; positively regulates GO:0036446 References: PMID:20533548 Sources: GOC:BHF, GOC:BHF_miRNA, GOC:TermGenie, GOC:rph, GO_REF:0000058 Definition: Any process that activates or increases the frequency, rate or extent of myofibroblast differentiation.